ribulose-1,5-bisphosphate carboxylase/oxygenase activator activity [GO:0046863] (molecular function) Also known as: ribulose-1,5-bisphosphate carboxylase/oxygenase activase activity, ribulose-bisphosphate carboxylase activase activity, rubisco activase activity, rubisco activator Relationships: is a type of GO:0008047; positively regulates ribulose-bisphosphate carboxylase activity [GO:0016984] References: PMID:10430961, PMID:10965036, PMID:2404515 Definition: Binds to and iincreases the activity of rubisco by the removal of otherwise inhibitory sugar phosphates: RuBP, and in some plants, 2-carboxyarabinitol 1-phosphate. Note: See also the molecular function term 'ribulose-bisphosphate carboxylase activity ; GO:0016984'.